{
  "term_label": "intracellular sodium ion homeostasis",
  "gene_name": "Sodium_potassium-transporting ATPase subunit alpha-4",
  "gene_symbol": "ATP1A4",
  "gene": "UniProtKB:Q13733",
  "term_id": "GO:0006883"
}